thiamine diphosphate phosphatase activity [GO:0004787] (molecular function) Also known as: thiamine diphosphatase activity, TPPase activity, thiamin pyrophosphatase activity, thiamin-pyrophosphatase activity, thiamine pyrophosphatase activity, thiamine-diphosphatase activity, thiaminpyrophosphatase activity Definition: Catalysis of the reaction: thiamine diphosphate + H2O = thiamine monophosphate + phosphate. Relationships: is a type of pyrophosphatase activity [GO:0016462] Sources: GOC:ai, RHEA:27998